purine alkaloid biosynthetic process [GO:0009711] (biological process) Definition: The chemical reactions and pathways resulting in the breakdown of purine alkaloids, compounds derived from purine and composed of an N-containing double ring structure. Sources: GOC:ai Also known as: purine alkaloid anabolism, purine alkaloid biosynthesis, purine alkaloid formation, purine alkaloid synthesis Relationships: is a type of alkaloid biosynthetic process [GO:0009821]; is a type of GO:0046446; is a type of purine-containing compound biosynthetic process [GO:0072522]